regulation of DNA catabolic process [GO:1903624] (BP) References: PMID:2001740 Sources: GOC:TermGenie, GO_REF:0000058 Definition: Any process that modulates the frequency, rate or extent of DNA catabolic process. Relationships: is a type of regulation of catabolic process [GO:0009894]; is a type of GO:0051052; regulates GO:0006308 Also known as: regulation of DNA breakdown, regulation of DNA catabolism, regulation of DNA degradation Subtypes: regulation of apoptotic DNA fragmentation [GO:1902510], negative regulation of DNA catabolic process [GO:1903625], positive regulation of DNA catabolic process [GO:1903626]